{
  "gene_name": "T-box transcription factor TBX21",
  "gene_symbol": "TBX21",
  "term_label": "DNA-binding transcription factor activity, RNA polymerase II-specific",
  "gene": "UniProtKB:Q9UL17",
  "term_id": "GO:0000981"
}